positive regulation of mitotic sister chromatid biorientation [GO:0140429] (biological process) Definition: Any process that activates or increases the frequency, rate or extent of mitotic sister chromatid biorientation, the mitotic cell cycle process in which sister chromatids establish stable, end-on attachments to the plus ends of microtubules emanating from opposite spindle poles, oriented such that separation can proceed. Also known as: correction of merotelic kinetochore attachment, mitotic, correction of mono-orientation defects, correction of syntelic kinetochore attachment, mitotic, repair of mitotic merotelic kinetochore attachment defect, repair of mitotic merotelic kinetochore attachment defects, repair of mitotic mono-orientation defect, repair of mitotic mono-orientation defects References: PMID:15525536, PMID:20739936, PMID:21306900 Sources: GOC:mtg_cell_cycle, GOC:vw Relationships: is a type of response to mitotic cell cycle spindle assembly checkpoint signaling [GO:0072479]; is_a repair of mitotic kinetochore microtubule attachment defect [GO:0140273]; is a type of GO:1902425; RO_0002213 mitotic sister chromatid biorientation [GO:1990758]